{
  "term_label": "extracellular matrix organization",
  "gene": "UniProtKB:Q03692",
  "gene_name": "Collagen alpha-1(X) chain",
  "term_id": "GO:0030198",
  "gene_symbol": "COL10A1"
}